{
  "gene_name": "Calicin",
  "gene_symbol": "CCIN",
  "gene": "UniProtKB:Q13939",
  "term_id": "GO:0043161",
  "term_label": "proteasome-mediated ubiquitin-dependent protein catabolic process"
}